{
  "term_label": "neuron differentiation",
  "gene_name": "Homeobox protein notochord",
  "gene": "UniProtKB:A8MTQ0",
  "term_id": "GO:0030182",
  "gene_symbol": "NOTO"
}